dynactin binding [GO:0034452] (MF) Definition: Binding to a dynactin complex; a large protein complex that activates dynein-based motor activity. Sources: GOC:BHF, GOC:mah Relationships: is a type of cytoskeletal protein binding [GO:0008092]